{
  "term_id": "GO:0035497",
  "gene_symbol": "CREB5",
  "term_label": "cAMP response element binding",
  "gene_name": "Cyclic AMP-responsive element-binding protein 5",
  "gene": "UniProtKB:Q02930"
}